{
  "term_label": "regulation of transcription by RNA polymerase II",
  "gene_symbol": "ZNF865",
  "gene_name": "Zinc finger protein 865",
  "gene": "UniProtKB:P0CJ78",
  "term_id": "GO:0006357"
}